terminal web [GO:1990357] (CC) Relationships: is a type of cortical actin cytoskeleton [GO:0030864] References: PMID:19437512, PMID:24677443, PMID:7511618 Sources: GOC:kmv, Wikipedia:Terminal_web Definition: An actin-rich cytoskeletal network located beneath the microvilli of the apical plasma membrane of polarized epithelial cells. In addition to actin filaments, the terminal web may contain actin-binding proteins, myosin motor proteins, and intermediate filaments. The terminal web can function as a contractile structure that influences the spatial distribution of microvilli as well as the development and morphogenesis of tissues containing polarized epithelial cells.